mitotic G1 cell size control checkpoint signaling [GO:0031568] (biological process) Sources: GOC:mtg_cell_cycle Also known as: mitotic G1 cell size control checkpoint, mitotic cell cycle G1/S transition size control checkpoint, G1 cell size control checkpoint, G1 cell size control checkpoint signalling, signal transduction involved in G1 cell size control checkpoint, signal transduction involved in mitotic cell cycle G1/S transition size control checkpoint Definition: A signal transduction process that contributes to a cell size control checkpoint during the G1/S transition of the cell cycle. Relationships: is a type of GO:0031567; is_a GO:2000134; happens during G1 phase [GO:0051318]